{
  "gene": "UniProtKB:Q8IWT0",
  "gene_symbol": "ZBTB8OS",
  "gene_name": "Protein archease",
  "term_label": "tRNA-splicing ligase complex",
  "term_id": "GO:0072669"
}